{
  "term_id": "GO:0008146",
  "gene_name": "Sulfotransferase 2A1",
  "gene": "UniProtKB:Q06520",
  "gene_symbol": "SULT2A1",
  "term_label": "sulfotransferase activity"
}